{
  "term_id": "GO:0005654",
  "term_label": "nucleoplasm",
  "gene_symbol": "NPM1",
  "gene": "UniProtKB:P06748",
  "gene_name": "Nucleophosmin"
}